atrial septum morphogenesis [GO:0060413] (biological process) Also known as: interatrial septum morphogenesis Relationships: is a type of cardiac septum morphogenesis [GO:0060411]; is part of GO:0003209; is part of atrial septum development [GO:0003283] Sources: GOC:dph, GOC:mtg_heart Subtypes: atrial septum primum morphogenesis [GO:0003289], GO:0003290, atrial septum intermedium morphogenesis [GO:0003291] Definition: The developmental process in which atrial septum is generated and organized. The atrial septum separates the upper chambers (the atria) of the heart from one another.